angioblast cell migration involved in selective angioblast sprouting [GO:0035475] (biological process) Regulation: regulated by regulation of angioblast cell migration involved in selective angioblast sprouting [GO:0035477] References: PMID:19815777 Sources: GOC:dgh Relationships: is a type of angioblast cell migration [GO:0035476]; is part of GO:0035474 Definition: The directional migration of angioblast cells as part of selective angioblast sprouting, which results in angioblast segregation into arterial and venous populations.